{
  "term_id": "UNKNOWN:0001",
  "term_label": "Unknown molecular function",
  "gene_name": "COMM domain-containing protein 10",
  "gene": "UniProtKB:Q9Y6G5",
  "gene_symbol": "COMMD10"
}